presynaptic active zone assembly [GO:1904071] (biological process) Regulation: regulated by regulation of presynaptic active zone assembly [GO:1905518]; negatively regulated by negative regulation of presynaptic active zone assembly [GO:1905519]; positively regulated by positive regulation of presynaptic active zone assembly [GO:1905520] Also known as: pre-synaptic active zone assembly, pre-synaptic active zone formation, presynaptic active zone formation, pre-synaptic active zone component assembly, pre-synaptic active zone component formation Definition: The aggregation, arrangement and bonding together of a set of components to form a presynaptic active zone. The presynaptic active zone is a specialized region of the plasma membrane and cell cortex of a presynaptic neuron; encompasses a region of the plasma membrane where synaptic vesicles dock and fuse, and a specialized cortical cytoskeletal matrix. References: PMID:10769383 Sources: GOC:TermGenie, GOC:pr, GO_REF:0000079 Relationships: is a type of cellular component assembly [GO:0022607]; is a type of GO:1990709; BFO_0000050 presynapse assembly [GO:0099054]